{
  "gene_name": "Ras-like protein family member 12",
  "term_id": "GO:0005886",
  "gene": "UniProtKB:Q9NYN1",
  "term_label": "plasma membrane",
  "gene_symbol": "RASL12"
}